purine deoxyribosyltransferase activity [GO:0044102] (molecular function) Relationships: is a type of GO:0016763 Also known as: purine 2'-deoxyribosyltransferase activity, PTD References: PMID:11836245 Sources: GOC:jl Definition: Catalysis of deoxyribose exchange between purine deoxyribonucleoside as a donor and purine base as an acceptor.